{
  "gene_name": "TNF receptor-associated factor 6",
  "term_label": "ubiquitin protein ligase activity",
  "gene": "UniProtKB:Q9Y4K3",
  "term_id": "GO:0061630",
  "gene_symbol": "TRAF6"
}